positive regulation of kinase activity [GO:0033674] (biological process) Relationships: is a type of positive regulation of phosphorylation [GO:0042327]; is a type of GO:0043085; is a type of GO:0043549; positively regulates kinase activity [GO:0016301] Also known as: up regulation of kinase activity, up-regulation of kinase activity, upregulation of kinase activity, kinase activator, stimulation of kinase activity Definition: Any process that activates or increases the frequency, rate or extent of kinase activity, the catalysis of the transfer of a phosphate group, usually from ATP, to a substrate molecule. Sources: GOC:mah Subtypes: positive regulation of protein kinase activity [GO:0045860], positive regulation of lipid kinase activity [GO:0090218], positive regulation of hexokinase activity [GO:1903301]